{
  "gene_symbol": "GUCA1B",
  "gene_name": "Guanylyl cyclase-activating protein 2",
  "term_label": "visual perception",
  "term_id": "GO:0007601",
  "gene": "UniProtKB:Q9UMX6"
}